negative regulation of venous endothelial cell fate commitment [GO:2000788] (biological process) References: PMID:11585794 Definition: Any process that stops, prevents or reduces the frequency, rate or extent of venous endothelial cell fate commitment. Relationships: is a type of GO:0010454; is a type of GO:0110059; is a type of GO:2000787; negatively regulates venous endothelial cell fate commitment [GO:0060845]